{
  "term_id": "UNKNOWN:0001",
  "term_label": "Unknown molecular function",
  "gene": "UniProtKB:Q9C0J8",
  "gene_name": "pre-mRNA 3' end processing protein WDR33",
  "gene_symbol": "WDR33"
}